{
  "gene_name": "Janus kinase and microtubule-interacting protein 3",
  "term_label": "Unknown molecular function",
  "term_id": "UNKNOWN:0001",
  "gene": "UniProtKB:Q5VZ66",
  "gene_symbol": "JAKMIP3"
}